mesenchyme migration involved in limb bud formation [GO:0090496] (biological process) Sources: GOC:dph, GOC:tb Relationships: is a type of GO:0090131; is part of limb bud formation [GO:0060174] Definition: The migration of mesenchymal tissue that contributes to the formation of a limb bud.